{
  "term_label": "signal transduction",
  "gene": "UniProtKB:Q9NUJ3",
  "gene_name": "T-complex protein 11-like protein 1",
  "gene_symbol": "TCP11L1",
  "term_id": "GO:0007165"
}